synonym_type_property [oboInOwl#SynonymTypeProperty]